{
  "gene": "UniProtKB:P52954",
  "term_label": "DNA-binding transcription factor activity, RNA polymerase II-specific",
  "gene_symbol": "LBX1",
  "gene_name": "Transcription factor LBX1",
  "term_id": "GO:0000981"
}